{
  "term_id": "UNKNOWN:0002",
  "gene_symbol": "TAF9B",
  "term_label": "Unknown biological process",
  "gene_name": "Transcription initiation factor TFIID subunit 9B",
  "gene": "UniProtKB:Q9HBM6"
}